rhythmic behavior [GO:0007622] (biological process) Relationships: is a type of behavior [GO:0007610] Definition: The specific behavior of an organism that recur with measured regularity. Sources: GOC:jl, GOC:pr Also known as: rhythmic behavioral response to stimulus, rhythmic behaviour, rhythmic behavioural response to stimulus Subtypes: GO:0048512